{
  "gene_symbol": "ZNF16",
  "gene": "UniProtKB:P17020",
  "gene_name": "Zinc finger protein 16",
  "term_label": "nucleus",
  "term_id": "GO:0005634"
}